{
  "term_id": "GO:0035313",
  "gene_symbol": "LRG1",
  "gene": "UniProtKB:P02750",
  "gene_name": "Leucine-rich alpha-2-glycoprotein",
  "term_label": "wound healing, spreading of epidermal cells"
}